{
  "term_id": "GO:0071805",
  "gene_symbol": "SLC9A3",
  "term_label": "potassium ion transmembrane transport",
  "gene_name": "Sodium_hydrogen exchanger 3",
  "gene": "UniProtKB:P48764"
}